{
  "gene": "UniProtKB:A0A075B7E0",
  "gene_name": "Protein IGHD3OR15-3A (Fragment)",
  "term_label": "Unknown molecular function",
  "gene_symbol": "IGHD3OR15-3B",
  "term_id": "UNKNOWN:0001"
}